{
  "gene_symbol": "POU1F1",
  "term_id": "UNKNOWN:0003",
  "term_label": "Unknown cellular component",
  "gene_name": "Pituitary-specific positive transcription factor 1",
  "gene": "UniProtKB:P28069"
}